{
  "term_id": "UNKNOWN:0001",
  "gene_symbol": "TEX55",
  "gene_name": "Testis-specific expressed protein 55",
  "gene": "UniProtKB:Q96M34",
  "term_label": "Unknown molecular function"
}